cycloartenol 24-C-methyltransferase activity [GO:0030796] (molecular function) Relationships: is a type of S-adenosylmethionine-dependent methyltransferase activity [GO:0008757] Sources: EC:2.1.1.142, RHEA:13137 Definition: Catalysis of the reaction: S-adenosyl-L-methionine + cycloartenol = (24R)-24-methylcycloart-25-en-3beta-ol + S-adenosyl-L-homocysteine + H+. Also known as: sterol C-methyltransferase activity, S-adenosyl-L-methionine:cycloartenol 24-C-methyltransferase activity